{
  "term_label": "Unknown cellular component",
  "term_id": "UNKNOWN:0003",
  "gene_symbol": "TCTE1",
  "gene_name": "Dynein regulatory complex subunit 5",
  "gene": "UniProtKB:Q5JU00"
}